{
  "gene": "UniProtKB:Q16518",
  "gene_symbol": "RPE65",
  "term_label": "retinol isomerase activity",
  "gene_name": "Retinoid isomerohydrolase",
  "term_id": "GO:0050251"
}